{
  "gene_name": "Ephrin type-A receptor 10",
  "gene_symbol": "EPHA10",
  "term_id": "GO:0007411",
  "gene": "UniProtKB:Q5JZY3",
  "term_label": "axon guidance"
}